{
  "gene": "UniProtKB:Q6I9Y2",
  "gene_symbol": "THOC7",
  "term_label": "Unknown molecular function",
  "gene_name": "THO complex subunit 7 homolog",
  "term_id": "UNKNOWN:0001"
}